{
  "term_id": "GO:0005634",
  "term_label": "nucleus",
  "gene_symbol": "RNF25",
  "gene_name": "E3 ubiquitin-protein ligase RNF25",
  "gene": "UniProtKB:Q96BH1"
}